{
  "term_label": "ATP binding",
  "gene_symbol": "ABCD1",
  "term_id": "GO:0005524",
  "gene_name": "ATP-binding cassette sub-family D member 1",
  "gene": "UniProtKB:P33897"
}